tocopherol cyclase activity [GO:0009976] (molecular function) References: PMID:12213958 Sources: EC:5.5.1.24 Regulation: regulated by GO:1902171 Definition: Catalysis of the reactions: delta-tocopherol = 2-methyl-6-phytyl-1,4-benzene-1,4-diol, gamma-tocopherol = 2,3-dimethyl-6-phytylbenzene-1,4-diol. delta-tocotrienol = 6-geranylgeranyl-2-methylbenzene-1,4-diol gamma-tocotrienol, and = 6-geranylgeranyl-2,3-dimethylbenzene-1,4-diol. Relationships: is a type of cyclase activity [GO:0009975]